{
  "gene_name": "Gamma-aminobutyric acid receptor subunit delta",
  "gene": "UniProtKB:O14764",
  "term_id": "GO:0004890",
  "gene_symbol": "GABRD",
  "term_label": "GABA-A receptor activity"
}